{
  "gene_symbol": "HLA-DQA1",
  "term_id": "GO:0019886",
  "gene_name": "HLA class II histocompatibility antigen, DQ alpha 1 chain",
  "term_label": "antigen processing and presentation of exogenous peptide antigen via MHC class II",
  "gene": "UniProtKB:P01909"
}